negative regulation of cellular response to X-ray [GO:2000684] (biological process) Relationships: is a type of negative regulation of cellular process [GO:0048523]; is a type of negative regulation of response to stimulus [GO:0048585]; is a type of regulation of cellular response to X-ray [GO:2000683]; negatively regulates GO:0071481 Also known as: negative regulation of cellular response to X-ray radiation stimulus Definition: Any process that stops, prevents or reduces the frequency, rate or extent of cellular response to X-ray. Sources: GOC:obol